negative regulation of proteoglycan biosynthetic process [GO:1902729] (BP) Definition: Any process that stops, prevents or reduces the frequency, rate or extent of the chemical reactions and pathways resulting in the formation of proteoglycans, any glycoprotein in which the carbohydrate units are glycosaminoglycans. References: PMID:23212449 Sources: GOC:TermGenie, GO_REF:0000058 Relationships: is a type of GO:0010561; negatively regulates proteoglycan biosynthetic process [GO:0030166] Also known as: down regulation of proteoglycan anabolism, down regulation of proteoglycan biosynthesis, down regulation of proteoglycan biosynthetic process, down regulation of proteoglycan formation, down regulation of proteoglycan synthesis, down-regulation of proteoglycan anabolism, down-regulation of proteoglycan biosynthesis, down-regulation of proteoglycan biosynthetic process, down-regulation of proteoglycan formation, down-regulation of proteoglycan synthesis, downregulation of proteoglycan anabolism, downregulation of proteoglycan biosynthesis, downregulation of proteoglycan biosynthetic process, downregulation of proteoglycan formation, downregulation of proteoglycan synthesis, negative regulation of proteoglycan anabolism, negative regulation of proteoglycan biosynthesis, negative regulation of proteoglycan formation, negative regulation of proteoglycan synthesis, inhibition of proteoglycan anabolism, inhibition of proteoglycan biosynthesis, inhibition of proteoglycan biosynthetic process, inhibition of proteoglycan formation, inhibition of proteoglycan synthesis